{
  "term_label": "inositol-1,3,4-trisphosphate 5-kinase activity",
  "gene_name": "Inositol-tetrakisphosphate 1-kinase",
  "gene_symbol": "ITPK1",
  "term_id": "GO:0052726",
  "gene": "UniProtKB:Q13572"
}